{
  "term_id": "GO:0017158",
  "gene": "UniProtKB:Q9H2B2",
  "term_label": "regulation of calcium ion-dependent exocytosis",
  "gene_name": "Synaptotagmin-4",
  "gene_symbol": "SYT4"
}